{
  "gene": "UniProtKB:P55851",
  "gene_symbol": "UCP2",
  "term_label": "mitochondrial inner membrane",
  "term_id": "GO:0005743",
  "gene_name": "Dicarboxylate carrier SLC25A8"
}